biotin--[biotin carboxyl-carrier protein] ligase activity [GO:0004077] (MF) Relationships: is a type of ligase activity, forming carbon-nitrogen bonds [GO:0016879]; is a type of catalytic activity, acting on a protein [GO:0140096] Definition: Catalysis of the reaction: ATP + biotin + L-lysyl-[protein] = AMP + diphosphate + H+ + N(6)-biotinyl-L-lysyl-[protein]. Sources: RHEA:11756 Also known as: biotin-acetyl-CoA carboxylase synthetase, biotin-protein ligase activity, HCS, acetyl CoA holocarboxylase synthetase activity, acetyl coenzyme A holocarboxylase synthetase activity, acetyl-CoA carboxylase biotin holoenzyme synthetase activity, biotin holoenzyme synthetase activity, biotin--[acetyl-CoA carboxylase] synthetase activity, biotin--protein ligase activity, biotin-acetyl coenzyme A carboxylase synthetase activity, biotin-acetyl-CoA-carboxylase ligase activity, biotin:apo-acetyl-CoA:carbon-dioxide ligase (ADP-forming) ligase (AMP-forming), biotin:apocarboxylase ligase activity